{
  "gene": "UniProtKB:Q16769",
  "gene_symbol": "QPCT",
  "gene_name": "Glutaminyl-peptide cyclotransferase",
  "term_label": "zinc ion binding",
  "term_id": "GO:0008270"
}